ornithine decarboxylase inhibitor activity [GO:0008073] (molecular function) Sources: GOC:jl Relationships: is a type of enzyme inhibitor activity [GO:0004857]; is_a ornithine decarboxylase regulator activity [GO:0042979]; negatively regulates ornithine decarboxylase activity [GO:0004586] Definition: Binds to and stops, prevents or reduces the activity of ornithine decarboxylase.